{
  "gene_name": "Contactin-associated protein-like 3",
  "gene_symbol": "CNTNAP3",
  "term_id": "GO:0007165",
  "term_label": "signal transduction",
  "gene": "UniProtKB:Q9BZ76"
}